{
  "gene_symbol": "KCNE2",
  "term_label": "regulation of ventricular cardiac muscle cell membrane repolarization",
  "gene": "UniProtKB:Q9Y6J6",
  "term_id": "GO:0060307",
  "gene_name": "Potassium voltage-gated channel subfamily E member 2"
}